positive regulation of mitotic spindle elongation [GO:1902846] (biological process) References: PMID:23087209 Sources: GOC:TermGenie, GO_REF:0000058 Definition: Any process that activates or increases the frequency, rate or extent of mitotic spindle elongation. Relationships: is a type of GO:0032888; is a type of positive regulation of mitotic sister chromatid segregation [GO:0062033]; positively regulates mitotic spindle elongation [GO:0000022] Also known as: positive regulation of spindle elongation during mitosis, up regulation of mitotic spindle elongation, up regulation of spindle elongation during mitosis, up-regulation of mitotic spindle elongation, up-regulation of spindle elongation during mitosis, upregulation of mitotic spindle elongation, upregulation of spindle elongation during mitosis, activation of mitotic spindle elongation, activation of spindle elongation during mitosis Subtypes: positive regulation of mitotic spindle elongation (spindle phase three) [GO:0110164]